heparan sulfate binding [GO:1904399] (molecular function) Relationships: is a type of GO:0005539; is a type of GO:0031406; is a type of sulfur compound binding [GO:1901681] References: PMID:8567685 Sources: GOC:TermGenie, GO_REF:0000067 Definition: Binding to heparan sulfate.